{
  "gene": "UniProtKB:P29466",
  "gene_symbol": "CASP1",
  "gene_name": "Caspase-1",
  "term_label": "positive regulation of apoptotic process",
  "term_id": "GO:0043065"
}